regulation of melanotic encapsulation of foreign target [GO:0140539] (biological process) Relationships: is a type of regulation of immune effector process [GO:0002697]; is a type of regulation of melanization defense response [GO:0035007]; regulates melanotic encapsulation of foreign target [GO:0035011] Definition: Any process that modulates the frequency, rate or extent of melanotic encapsulation of foreign target. Subtypes: GO:0140540 References: PMID:15749104, PMID:18457993